leading edge of axonal growth cone [GO:0061916] (cellular component) References: PMID:16098134 Definition: That part of the axonal growth cone which represents the distal part of the structure. Relationships: is a type of GO:0061850; is part of axonal growth cone [GO:0044295] Also known as: axonal growth cone leading edge, distal tip of axonal growth cone